{
  "gene_name": "BLOC-1-related complex subunit 8",
  "term_id": "UNKNOWN:0001",
  "term_label": "Unknown molecular function",
  "gene_symbol": "BORCS8",
  "gene": "UniProtKB:Q96FH0"
}